propionate catabolic process, 2-methylcitrate cycle [GO:0019629] (BP) Definition: The chemical reactions and pathways resulting in the breakdown of propionate that occurs in the 2-methylcitrate cycle. Sources: GOC:go_curators Relationships: is a type of propionate catabolic process [GO:0019543] Also known as: propionate breakdown, 2-methylcitrate cycle, propionate degradation, 2-methylcitrate cycle